{
  "term_label": "nucleus",
  "term_id": "GO:0005634",
  "gene_name": "Fez family zinc finger protein 2",
  "gene": "UniProtKB:Q8TBJ5",
  "gene_symbol": "FEZF2"
}